broken chromosome clustering [GO:0141112] (biological process) Relationships: is a type of chromosome organization [GO:0051276]; is part of DNA damage response [GO:0006974] Definition: The process of bringing together chromosomes fragments resulting from DNA damage. Broken chromosome tethering during mitosis ensures clustered segregation of the fragments to a single daughter cell nucleus, facilitating re-ligation with limited chromosome scattering and loss and enhancing genome integrity. References: PMID:37165191, PMID:37316668